{
  "gene_name": "Zinc finger protein 766",
  "gene": "UniProtKB:Q5HY98",
  "gene_symbol": "ZNF766",
  "term_label": "RNA polymerase II cis-regulatory region sequence-specific DNA binding",
  "term_id": "GO:0000978"
}